{
  "term_id": "GO:0000981",
  "gene_symbol": "NFATC1",
  "gene": "UniProtKB:O95644",
  "term_label": "DNA-binding transcription factor activity, RNA polymerase II-specific",
  "gene_name": "Nuclear factor of activated T-cells, cytoplasmic 1"
}